{
  "term_id": "GO:0000785",
  "gene": "UniProtKB:Q9UGL1",
  "term_label": "chromatin",
  "gene_symbol": "KDM5B",
  "gene_name": "Lysine-specific demethylase 5B"
}